{
  "gene_name": "Charged multivesicular body protein 5",
  "term_label": "late endosome to vacuole transport via multivesicular body sorting pathway",
  "gene": "UniProtKB:Q9NZZ3",
  "term_id": "GO:0032511",
  "gene_symbol": "CHMP5"
}